{
  "gene_name": "Inhibin beta A chain",
  "gene_symbol": "INHBA",
  "gene": "UniProtKB:P08476",
  "term_label": "cytokine activity",
  "term_id": "GO:0005125"
}